{
  "gene": "UniProtKB:P04406",
  "term_id": "GO:0004365",
  "gene_symbol": "GAPDH",
  "gene_name": "Glyceraldehyde-3-phosphate dehydrogenase",
  "term_label": "glyceraldehyde-3-phosphate dehydrogenase (NAD+) (phosphorylating) activity"
}